{
  "term_id": "GO:0001096",
  "term_label": "TFIIF-class transcription factor complex binding",
  "gene_name": "General transcription factor IIF subunit 1",
  "gene_symbol": "GTF2F1",
  "gene": "UniProtKB:P35269"
}